tRNA import into nucleus [GO:0035719] (biological process) Definition: The directed movement of tRNA from the cytoplasm to the nucleus. Relationships: is a type of GO:0006404; is a type of tRNA transport [GO:0051031] References: PMID:20032305 Sources: GOC:vw Also known as: retrograde tRNA transport into nucleus, tRNA nuclear import